{
  "gene_symbol": "HIF1A",
  "gene_name": "Hypoxia-inducible factor 1-alpha",
  "gene": "UniProtKB:Q16665",
  "term_id": "GO:0005634",
  "term_label": "nucleus"
}